{
  "term_label": "dendrite",
  "gene": "UniProtKB:Q92953",
  "term_id": "GO:0030425",
  "gene_symbol": "KCNB2",
  "gene_name": "Potassium voltage-gated channel subfamily B member 2"
}